{
  "gene": "UniProtKB:Q8N9R8",
  "term_id": "GO:0003714",
  "term_label": "transcription corepressor activity",
  "gene_symbol": "SCAI",
  "gene_name": "Protein SCAI"
}